{
  "gene": "UniProtKB:Q9UI46",
  "term_label": "outer dynein arm",
  "gene_name": "Dynein axonemal intermediate chain 1",
  "gene_symbol": "DNAI1",
  "term_id": "GO:0036157"
}